{
  "gene": "UniProtKB:Q8N8D9",
  "gene_name": "Uncharacterized protein IRF1-AS1",
  "gene_symbol": "IRF1-AS1",
  "term_label": "Unknown biological process",
  "term_id": "UNKNOWN:0002"
}